sequestering of extracellular ligand from receptor [GO:0035581] (biological process) Note: Preventing a ligand from binding to its cell surface receptor be achieved by binding to the ligand directly, or by binding to members of a ligand-containing complex. Sources: GOC:BHF, GOC:signaling Subtypes: sequestering of BMP in extracellular matrix [GO:0035582], sequestering of TGFbeta in extracellular matrix [GO:0035583], sequestering of BMP from receptor via BMP binding [GO:0038098], GO:0038101, sequestering of TGFbeta from receptor via TGFbeta binding [GO:0038105] Also known as: extracellular sequestering of receptor ligand, negative regulation of protein bioavailability Relationships: is a type of GO:1900116 Definition: The process of binding or confining an extracellular signaling ligand, such that the ligand is unable to bind to its cell surface receptor.